amino acid:sodium symporter activity [GO:0005283] (molecular function) Definition: Enables the transfer of a solute or solutes from one side of a membrane to the other according to the reaction: amino acid(out) + Na+(out) = amino acid(in) + Na+(in). Relationships: is a type of amino acid:monoatomic cation symporter activity [GO:0005416]; is a type of solute:sodium symporter activity [GO:0015370] Also known as: sodium/amino acid transporter activity, sodium/excitatory amino acid cotransporter activity, sodium:amino acid transporter activity, sodium/excitatory amino acid symporter activity, sodium:amino acid symporter activity, glutamate/aspartate:sodium symporter activity, insulin-activated sodium/amino acid transporter activity, insulin-activated sodium:amino acid symporter activity, insulin-activated sodium:amino acid transporter activity, isoleucine/valine:sodium symporter activity, threonine/serine:sodium symporter activity Sources: GOC:ai Subtypes: neutral L-amino acid:sodium symporter activity [GO:0005295], GO:0005298, gamma-aminobutyric acid:sodium:chloride symporter activity [GO:0005332], neutral, basic amino acid:sodium:chloride symporter activity [GO:0015374], glutamate:sodium symporter activity [GO:0015501], GO:0015655, GO:0140931